oligopeptide transmembrane transport [GO:0035672] (biological process) Relationships: is a type of oligopeptide transport [GO:0006857]; is a type of transmembrane transport [GO:0055085] Sources: GOC:vw, ISBN:0198506732 Note: Note that this term is not intended for use in annotating lateral movement within membranes. Subtypes: dipeptide transmembrane transport [GO:0035442], GO:0035443, phytochelatin 2 import into vacuole [GO:0036246], phytochelatin 3 import into vacuole [GO:0036247], GO:0036248, GO:0090374, oligopeptide import across plasma membrane [GO:0140205] Also known as: oligopeptide membrane transport Definition: The process in which an oligopeptide is transported across a membrane. Oligopeptides are molecules that contain a small number (2 to 20) of amino-acid residues connected by peptide linkages.